{
  "gene_symbol": "TRH",
  "term_id": "GO:0008437",
  "gene_name": "Pro-thyrotropin-releasing hormone",
  "term_label": "thyrotropin-releasing hormone activity",
  "gene": "UniProtKB:P20396"
}